3-hydroxy-2-methylbutyryl-CoA dehydrogenase activity [GO:0047015] (molecular function) Definition: Catalysis of the reaction: NAD+ + 2-methyl-3-hydroxybutyryl-CoA = NADH + H+ + 2-methylaceto-acetyl-CoA. Sources: EC:1.1.1.178, MetaCyc:1.1.1.178-RXN Also known as: (2S,3S)-3-hydroxy-2-methylbutanoyl-CoA:NAD+ oxidoreductase activity, 2-methyl-3-hydroxy-butyryl CoA dehydrogenase activity, 2-methyl-3-hydroxybutyryl coenzyme A dehydrogenase activity, 2-methyl-3-hydroxybutyryl-CoA dehydrogenase activity Relationships: is a type of oxidoreductase activity, acting on the CH-OH group of donors, NAD or NADP as acceptor [GO:0016616]